CARD domain binding [GO:0050700] (molecular function) References: PMID:12054670 Definition: Binding to a CARD (N-terminal caspase recruitment) domain, a protein-protein interaction domain that belongs to the death domain-fold superfamily. These protein molecule families are similar in structure with each consisting of six or seven anti-parallel alpha-helices that form highly specific homophilic interactions between signaling partners. CARD exists in the N-terminal prodomains of several caspases and in apoptosis-regulatory proteins and mediates the assembly of CARD-containing proteins that participate in activation or suppression of CARD carrying members of the caspase family. Relationships: is a type of protein domain specific binding [GO:0019904]